{
  "gene_symbol": "RBM3",
  "term_id": "GO:0043023",
  "term_label": "ribosomal large subunit binding",
  "gene_name": "RNA-binding protein 3",
  "gene": "UniProtKB:P98179"
}